cotranslational protein targeting to membrane [GO:0006613] (biological process) Definition: The targeting of proteins to a membrane that occurs during translation. The transport of most secretory proteins, particularly those with more than 100 amino acids, into the endoplasmic reticulum lumen occurs in this manner, as does the import of some proteins into mitochondria. Relationships: is a type of GO:0006612 Subtypes: SRP-dependent cotranslational protein targeting to membrane [GO:0006614] References: PMID:10512867, PMID:16896215 Sources: ISBN:0716731363 Also known as: cotranslational membrane targeting, cotranslational protein membrane targeting, cotranslational protein-membrane targeting